{
  "term_id": "GO:0005886",
  "gene": "UniProtKB:Q07912",
  "term_label": "plasma membrane",
  "gene_symbol": "TNK2",
  "gene_name": "Activated CDC42 kinase 1"
}